{
  "term_label": "lactose binding",
  "gene_symbol": "LGALS1",
  "term_id": "GO:0030395",
  "gene_name": "Galectin-1",
  "gene": "UniProtKB:P09382"
}